regulation of transferase activity [GO:0051338] (biological process) Note: This term is useful for grouping, but is too general for manual annotation. Please use a child term instead. Sources: GOC:ai Subtypes: GO:0010835, regulation of kinase activity [GO:0043549], GO:0051438, positive regulation of protein-glutamine gamma-glutamyltransferase activity [GO:0150074], GO:1900260, positive regulation of DNA-directed DNA polymerase activity [GO:1900264], GO:1903302, positive regulation of serine C-palmitoyltransferase activity [GO:1904222], negative regulation of polynucleotide adenylyltransferase activity [GO:1904246], GO:1904247, regulation of glycogen (starch) synthase activity [GO:2000465], regulation of ATP citrate synthase activity [GO:2000983] Relationships: is a type of regulation of catalytic activity [GO:0050790]; regulates transferase activity [GO:0016740] Definition: Any process that modulates the frequency, rate or extent of transferase activity, the catalysis of the transfer of a group, e.g. a methyl group, glycosyl group, acyl group, phosphorus-containing, or other groups, from one compound (generally regarded as the donor) to another compound (generally regarded as the acceptor). Transferase is the systematic name for any enzyme of EC class 2. Also known as: transferase regulator